{
  "gene_name": "Rho GTPase-activating protein 32",
  "term_label": "small GTPase-mediated signal transduction",
  "term_id": "GO:0007264",
  "gene": "UniProtKB:A7KAX9",
  "gene_symbol": "ARHGAP32"
}